{
  "term_label": "RNA stabilization",
  "gene": "UniProtKB:Q9NP64",
  "gene_name": "Zinc finger CCHC domain-containing protein 17",
  "gene_symbol": "ZCCHC17",
  "term_id": "GO:0043489"
}